{
  "gene": "UniProtKB:Q14393",
  "term_id": "GO:0051897",
  "term_label": "positive regulation of phosphatidylinositol 3-kinase/protein kinase B signal transduction",
  "gene_symbol": "GAS6",
  "gene_name": "Growth arrest-specific protein 6"
}